{
  "gene_symbol": "CCDC191",
  "term_label": "Unknown cellular component",
  "gene": "UniProtKB:Q8NCU4",
  "gene_name": "Coiled-coil domain-containing protein 191",
  "term_id": "UNKNOWN:0003"
}